{
  "gene_symbol": "TOP1MT",
  "term_id": "GO:0003917",
  "gene": "UniProtKB:Q969P6",
  "term_label": "DNA topoisomerase type I (single strand cut, ATP-independent) activity",
  "gene_name": "DNA topoisomerase I, mitochondrial"
}